oxidoreductase activity, acting on the CH-NH2 group of donors [GO:0016638] (molecular function) Sources: EC:1.4.-.-, GOC:ai Also known as: oxidoreductase activity, acting on the CH-NH2 group of donors, other acceptors Definition: Catalysis of an oxidation-reduction (redox) reaction in which a CH-NH2 group acts as a hydrogen or electron donor and reduces a hydrogen or electron acceptor. Subtypes: alanine dehydrogenase activity [GO:0000286], GO:0008718, glutamate synthase activity [GO:0015930], oxidoreductase activity, acting on the CH-NH2 group of donors, NAD or NADP as acceptor [GO:0016639], oxidoreductase activity, acting on the CH-NH2 group of donors, cytochrome as acceptor [GO:0016640], GO:0016641, oxidoreductase activity, acting on the CH-NH2 group of donors, disulfide as acceptor [GO:0016642], oxidoreductase activity, acting on the CH-NH2 group of donors, iron-sulfur protein as acceptor [GO:0016643], GO:0030058, aspartate dehydrogenase [NAD(P)+] activity [GO:0033735], GO:0034557, taurine dehydrogenase activity [GO:0050323], glycine dehydrogenase (cyanide-forming) activity [GO:0050622], oxidoreductase activity, acting on the CH-NH2 group of donors, with a copper protein as acceptor [GO:0052877] Relationships: is a type of oxidoreductase activity [GO:0016491]